{
  "term_label": "regulation of transcription by RNA polymerase II",
  "gene_name": "Zinc finger protein 124",
  "gene_symbol": "ZNF124",
  "term_id": "GO:0006357",
  "gene": "UniProtKB:Q15973"
}